{
  "gene_symbol": "EPGN",
  "term_label": "growth factor activity",
  "term_id": "GO:0008083",
  "gene_name": "Epigen",
  "gene": "UniProtKB:Q6UW88"
}